{
  "term_label": "protein import into peroxisome matrix, docking",
  "gene_symbol": "PEX13",
  "term_id": "GO:0016560",
  "gene_name": "Peroxisomal membrane protein PEX13",
  "gene": "UniProtKB:Q92968"
}